{
  "gene_name": "Chromatin-remodeling ATPase INO80",
  "gene": "UniProtKB:Q9ULG1",
  "term_id": "GO:0016887",
  "term_label": "ATP hydrolysis activity",
  "gene_symbol": "INO80"
}